regulation of response to G1 DNA damage checkpoint signaling [GO:1902155] (biological process) Subtypes: GO:1902156 Relationships: is a type of regulation of response to DNA damage checkpoint signaling [GO:1902153]; regulates response to G1 DNA damage checkpoint signaling [GO:0072432] Definition: Any process that modulates the frequency, rate or extent of response to G1 DNA damage checkpoint signaling. Sources: GOC:TermGenie, GOC:mtg_cell_cycle Also known as: regulation of mitotic cell cycle G1/S transition DNA damage checkpoint effector process, regulation of response to mitotic cell cycle G1/S transition DNA damage checkpoint signaling, regulation of response to signal involved in mitotic cell cycle G1/S transition DNA damage checkpoint